taste bud morphogenesis [GO:0061194] (biological process) Definition: The process in which the anatomical structures of the taste bud are generated and organized. The taste bud is a specialized area of the tongue that contains taste receptors. Sources: GOC:dph Relationships: is a type of sensory organ morphogenesis [GO:0090596]; is part of tongue morphogenesis [GO:0043587]; is part of GO:0061193